{
  "term_id": "GO:0004925",
  "gene_symbol": "IL23R",
  "gene_name": "Interleukin-23 receptor",
  "gene": "UniProtKB:Q5VWK5",
  "term_label": "prolactin receptor activity"
}